{
  "gene_name": "Bleomycin hydrolase",
  "term_id": "GO:0005737",
  "gene_symbol": "BLMH",
  "gene": "UniProtKB:Q13867",
  "term_label": "cytoplasm"
}